{
  "gene_name": "Serine_threonine-protein phosphatase 2A activator",
  "gene_symbol": "PTPA",
  "term_label": "protein tyrosine phosphatase activator activity",
  "gene": "UniProtKB:Q15257",
  "term_id": "GO:0008160"
}